hindgut development [GO:0061525] (biological process) Relationships: is a type of digestive tract development [GO:0048565] Sources: GOC:dph Definition: The process whose specific outcome is the progression of the hindgut over time, from its formation to the mature structure. The hindgut is part of the alimentary canal that lies posterior to the midgut.